sulfur dioxygenase activity [GO:0050313] (molecular function) Definition: Catalysis of the reaction: S-sulfanylglutathione + O2 + H2O = sulfite + glutathione + 2 H+. Sources: EC:1.13.11.18 Also known as: sulphur dioxygenase activity, S-sulfanylglutathione:oxygen oxidoreductase activity, sulfur oxygenase activity, sulfur:oxygen oxidoreductase activity Relationships: is a type of oxidoreductase activity, acting on single donors with incorporation of molecular oxygen, incorporation of two atoms of oxygen [GO:0016702]